{
  "term_id": "GO:0050650",
  "gene": "UniProtKB:Q8TE99",
  "term_label": "chondroitin sulfate proteoglycan biosynthetic process",
  "gene_name": "2-phosphoxylose phosphatase 1",
  "gene_symbol": "PXYLP1"
}